{
  "gene": "UniProtKB:P13073",
  "term_id": "UNKNOWN:0001",
  "term_label": "Unknown molecular function",
  "gene_symbol": "COX4I1",
  "gene_name": "Cytochrome c oxidase subunit 4 isoform 1, mitochondrial"
}